{
  "gene_symbol": "LIPC",
  "gene": "UniProtKB:P11150",
  "gene_name": "Hepatic triacylglycerol lipase",
  "term_id": "GO:0019433",
  "term_label": "triglyceride catabolic process"
}